{
  "term_label": "Unknown molecular function",
  "gene_symbol": "AKAIN1",
  "term_id": "UNKNOWN:0001",
  "gene_name": "A-kinase anchor protein inhibitor 1",
  "gene": "UniProtKB:P0CW23"
}